{
  "term_label": "Unknown biological process",
  "gene_symbol": "C20orf141",
  "gene": "UniProtKB:Q9NUB4",
  "gene_name": "Uncharacterized protein C20orf141",
  "term_id": "UNKNOWN:0002"
}